{
  "gene": "UniProtKB:Q7Z6M2",
  "term_id": "GO:0031398",
  "gene_symbol": "FBXO33",
  "term_label": "positive regulation of protein ubiquitination",
  "gene_name": "F-box only protein 33"
}